{
  "term_label": "Unknown molecular function",
  "term_id": "UNKNOWN:0001",
  "gene_symbol": "KRTAP10-2",
  "gene": "UniProtKB:P60368",
  "gene_name": "Keratin-associated protein 10-2"
}